regulation of biosynthetic process [GO:0009889] (biological process) Sources: GOC:go_curators Definition: Any process that modulates the frequency, rate or extent of the chemical reactions and pathways resulting in the formation of substances. Subtypes: GO:0009890, positive regulation of biosynthetic process [GO:0009891], GO:0009962, regulation of macromolecule biosynthetic process [GO:0010556], regulation of ketone biosynthetic process [GO:0010566], GO:0010967, GO:0030808, GO:0032965, GO:0043255, regulation of poly(3-hydroxyalkanoate) biosynthetic process [GO:0043286], regulation of nitric oxide biosynthetic process [GO:0045428], regulation of hormone biosynthetic process [GO:0046885], regulation of lipid biosynthetic process [GO:0046890], regulation of acyl-CoA biosynthetic process [GO:0050812], regulation of adenine biosynthetic process [GO:0061934], regulation of taurine biosynthetic process [GO:0062089], GO:0062161, regulation of thiamine diphosphate biosynthetic process [GO:0070616], regulation of coenzyme A biosynthetic process [GO:0080020], regulation of photorespiration [GO:0080093], regulation of salicylic acid biosynthetic process [GO:0080142], regulation of (R)-mevalonic acid biosynthetic process [GO:0106107], regulation of UDP-N-acetylglucosamine biosynthetic process [GO:0106278], GO:1900351, regulation of secondary metabolite biosynthetic process [GO:1900376], regulation of austinol biosynthetic process [GO:1900640], regulation of pseurotin A biosynthetic process [GO:1900849], regulation of hexadecanal biosynthetic process [GO:1900902], regulation of olefin biosynthetic process [GO:1900911], regulation of methanophenazine biosynthetic process [GO:1900962], regulation of sarcinapterin biosynthetic process [GO:1900971], regulation of tatiopterin biosynthetic process [GO:1900974], regulation of phenazine biosynthetic process [GO:1900980], GO:1901463, GO:1901577, regulation of fumagillin biosynthetic process [GO:1902090], regulation of alcohol biosynthetic process [GO:1902930], regulation of dopamine biosynthetic process [GO:1903179], GO:1903426, GO:1903786, regulation of pyrimidine-containing compound salvage [GO:1903930], regulation of hydrogen sulfide biosynthetic process [GO:1904826], regulation of vitamin E biosynthetic process [GO:1904965], regulation of quinolinate biosynthetic process [GO:1904984], regulation of serotonin biosynthetic process [GO:1905627], GO:1905722, regulation of acetylcholine biosynthetic process [GO:1905921], GO:2000282 Relationships: is a type of regulation of metabolic process [GO:0019222]; RO_0002211 biosynthetic process [GO:0009058] Also known as: regulation of anabolism, regulation of biosynthesis, regulation of formation, regulation of synthesis